flavonol-3-O-glucoside L-rhamnosyltransferase activity [GO:0047230] (molecular function) Relationships: is a type of UDP-glycosyltransferase activity [GO:0008194]; is a type of hexosyltransferase activity [GO:0016758] Sources: EC:2.4.1.159, MetaCyc:2.4.1.159-RXN Definition: Catalysis of the reaction: flavonol 3-O-D-glucoside + UDP-L-rhamnose = flavonol 3-O-L-rhamnosylglucoside + UDP. Also known as: UDP-L-rhamnose:flavonol-3-O-D-glucoside 6''-O-L-rhamnosyltransferase activity, UDP-rhamnose:flavonol 3-O-glucoside rhamnosyltransferase activity, uridine diphosphorhamnose-flavonol 3-O-glucoside rhamnosyltransferase activity